{
  "gene_name": "Kinase suppressor of Ras 1",
  "gene": "UniProtKB:Q8IVT5",
  "term_id": "GO:0016020",
  "term_label": "membrane",
  "gene_symbol": "KSR1"
}